positive regulation of mitochondrial DNA replication [GO:0090297] (biological process) Also known as: positive regulation of mitochondrial DNA synthesis Definition: Any process that increases the rate, frequency or extent of the process in which new strands of DNA are synthesized in the mitochondrion. Sources: GOC:tb Relationships: is a type of regulation of mitochondrial DNA replication [GO:0090296]; is a type of positive regulation of mitochondrial DNA metabolic process [GO:1901860]; is a type of GO:2000105; positively regulates mitochondrial DNA replication [GO:0006264]